response to genistein [GO:0033595] (biological process) Sources: GOC:mah Definition: Any process that results in a change in state or activity of a cell or an organism (in terms of movement, secretion, enzyme production, gene expression, etc.) as a result of a genistein stimulus. Subtypes: cellular response to genistein [GO:0071412] Relationships: is a type of response to hydroxyisoflavone [GO:0033594]